{
  "gene": "UniProtKB:Q99873",
  "gene_symbol": "PRMT1",
  "term_label": "protein-arginine omega-N monomethyltransferase activity",
  "gene_name": "Protein arginine N-methyltransferase 1",
  "term_id": "GO:0035241"
}